{
  "term_id": "GO:0001867",
  "gene_symbol": "FCN2",
  "term_label": "complement activation, lectin pathway",
  "gene": "UniProtKB:Q15485",
  "gene_name": "Ficolin-2"
}